{
  "gene": "UniProtKB:Q7Z494",
  "term_id": "GO:0001822",
  "gene_symbol": "NPHP3",
  "gene_name": "Nephrocystin-3",
  "term_label": "kidney development"
}